{
  "gene_symbol": "DDX60L",
  "term_label": "defense response to virus",
  "term_id": "GO:0051607",
  "gene": "UniProtKB:Q5H9U9",
  "gene_name": "Probable ATP-dependent RNA helicase DDX60-like"
}